{
  "term_id": "GO:0005886",
  "gene": "UniProtKB:Q8NGT1",
  "gene_symbol": "OR2K2",
  "gene_name": "Olfactory receptor 2K2",
  "term_label": "plasma membrane"
}